{
  "term_id": "GO:0005847",
  "gene_symbol": "SYMPK",
  "term_label": "mRNA cleavage and polyadenylation specificity factor complex",
  "gene_name": "Symplekin",
  "gene": "UniProtKB:Q92797"
}